{
  "gene_symbol": "PSMA8",
  "gene_name": "Proteasome subunit alpha-type 8",
  "term_label": "proteasome-mediated ubiquitin-dependent protein catabolic process",
  "term_id": "GO:0043161",
  "gene": "UniProtKB:Q8TAA3"
}